{
  "term_id": "GO:0005634",
  "term_label": "nucleus",
  "gene_name": "Serine_threonine-protein kinase Chk2",
  "gene": "UniProtKB:O96017",
  "gene_symbol": "CHEK2"
}